{
  "gene": "UniProtKB:Q9NQQ7",
  "gene_name": "Solute carrier family 35 member C2",
  "term_label": "UDP-glucose transmembrane transport",
  "gene_symbol": "SLC35C2",
  "term_id": "GO:0015786"
}